regulation of shoot apical meristem development [GO:1902183] (biological process) Definition: Any process that modulates the frequency, rate or extent of shoot apical meristem development. References: PMID:21496644 Sources: GOC:TermGenie Also known as: regulation of promeristem development, regulation of SAM development, regulation of primary shoot meristem development Relationships: is_a regulation of meristem development [GO:0048509]; regulates shoot apical meristem development [GO:1902182] Subtypes: negative regulation of shoot apical meristem development [GO:1902184], positive regulation of shoot apical meristem development [GO:1902185]